maturation of 4.5S rRNA [GO:0000476] (biological process) Sources: GOC:curators Relationships: is a type of rRNA processing [GO:0006364] Definition: Any process involved in the maturation of a precursor 4.5S ribosomal RNA (rRNA) molecule into a mature 4.5S rRNA molecule.